{
  "term_id": "GO:0007411",
  "term_label": "axon guidance",
  "gene_name": "Neuropilin-2",
  "gene_symbol": "NRP2",
  "gene": "UniProtKB:O60462"
}